oxidoreductase activity, acting on the CH-NH2 group of donors, oxygen as acceptor [GO:0016641] (molecular function) Definition: Catalysis of an oxidation-reduction (redox) reaction in which a CH-NH2 group acts as a hydrogen or electron donor and reduces an oxygen molecule. Sources: GOC:ai Relationships: is a type of oxidoreductase activity, acting on the CH-NH2 group of donors [GO:0016638] Subtypes: pyridoxamine phosphate oxidase activity [GO:0004733], GO:0008131, aliphatic amine oxidase activity [GO:0052595], GO:0052597, GO:0097621